lipid tube assembly involved in organelle fission [GO:0060990] (biological process) Also known as: lipid tubulation involved in organelle fission Definition: The aggregation, arrangement and bonding together of a set of macromolecules to form a macromolecular complex that contains a tube of lipid surrounded by a protein coat involved in membrane shaping of vesicle membranes as organelles undergo fission. Relationships: is a type of lipid tube assembly [GO:0060988]; is part of organelle fission [GO:0048285] Sources: GOC:ascb_2009, GOC:dph, GOC:tb